{
  "gene": "UniProtKB:Q5QJ38",
  "term_id": "UNKNOWN:0001",
  "gene_symbol": "TCHHL1",
  "gene_name": "Trichohyalin-like protein 1",
  "term_label": "Unknown molecular function"
}